{
  "gene": "UniProtKB:P56277",
  "gene_name": "Cx9C motif-containing protein 4",
  "term_id": "GO:0005758",
  "term_label": "mitochondrial intermembrane space",
  "gene_symbol": "CMC4"
}